RNA localization to Cajal body [GO:0090670] (biological process) Relationships: is_a GO:0090685 Definition: A process in which an RNA is transported to, or maintained in, a Cajal body. References: PMID:25467444 Sources: GOC:BHF, GOC:BHF_telomere, GOC:nc Subtypes: snRNA localization to Cajal body [GO:0061016], scaRNA localization to Cajal body [GO:0090666], telomerase RNA localization to Cajal body [GO:0090671]